petal epidermis patterning [GO:0080172] (BP) Definition: The regionalization process that regulates the coordinated growth and establishes the non-random spatial arrangement of the cells in the petal epidermis. Sources: GOC:tb Relationships: is a type of regionalization [GO:0003002]